{
  "gene_symbol": "SPDYC",
  "term_id": "GO:0019901",
  "gene": "UniProtKB:Q5MJ68",
  "term_label": "protein kinase binding",
  "gene_name": "Speedy protein C"
}